{
  "term_id": "UNKNOWN:0001",
  "gene_name": "Sperm-egg fusion protein LLCFC1",
  "gene_symbol": "LLCFC1",
  "term_label": "Unknown molecular function",
  "gene": "UniProtKB:Q96L11"
}